{
  "term_id": "GO:0007399",
  "term_label": "nervous system development",
  "gene_name": "Chondroitin sulfate proteoglycan 4",
  "gene": "UniProtKB:Q6UVK1",
  "gene_symbol": "CSPG4"
}